guanine catabolic process [GO:0006147] (biological process) Also known as: guanine breakdown, guanine catabolism, guanine degradation Sources: GOC:go_curators Definition: The chemical reactions and pathways resulting in the breakdown of guanine, 2-amino-6-hydroxypurine, a purine that is one of the five main bases found in nucleic acids and a component of a number of phosphorylated guanosine derivatives whose metabolic or regulatory functions are important. Relationships: is a type of GO:0006145; is a type of guanine metabolic process [GO:0046098]